{
  "gene_symbol": "MYOG",
  "gene": "UniProtKB:P15173",
  "term_id": "GO:0045663",
  "term_label": "positive regulation of myoblast differentiation",
  "gene_name": "Myogenin"
}